intronic snoRNA processing [GO:0031070] (biological process) Relationships: is a type of sno(s)RNA processing [GO:0043144] Definition: The biogenesis of a snoRNA molecule which resides within, and is processed from, the intron of a pre-mRNA. Subtypes: intronic box C/D snoRNA processing [GO:0034965], intronic box H/ACA snoRNA processing [GO:0034966] Sources: GOC:vw